negative regulation of formation of growth cone in injured axon [GO:1905943] (biological process) Definition: Any process that stops, prevents or reduces the frequency, rate or extent of formation of growth cone in injured axon. References: PMID:19737525 Sources: GOC:TermGenie, GO_REF:0000058 Also known as: down regulation of formation of growth cone in injured axon, down-regulation of formation of growth cone in injured axon, downregulation of formation of growth cone in injured axon, inhibition of formation of growth cone in injured axon Relationships: is a type of GO:0048688; is a type of regulation of formation of growth cone in injured axon [GO:1905942]; negatively regulates formation of growth cone in injured axon [GO:0048689]